{
  "gene": "UniProtKB:P01241",
  "gene_symbol": "GH1",
  "gene_name": "Somatotropin",
  "term_label": "extracellular space",
  "term_id": "GO:0005615"
}